alpha1-beta1 integrin-tissue transglutaminase complex [GO:0071091] (cellular component) References: PMID:10684262 Also known as: ITGA1-ITGB1-TGM2 complex Definition: A protein complex that consists of an alpha1-beta1 integrin complex bound to tissue transglutaminase. Relationships: is_a plasma membrane protein complex [GO:0098797]; is a type of catalytic complex [GO:1902494]